positive regulation of ethylene biosynthetic process [GO:0010365] (biological process) Relationships: is a type of regulation of ethylene biosynthetic process [GO:0010364]; is a type of positive regulation of olefin biosynthetic process [GO:1900913]; positively regulates ethylene biosynthetic process [GO:0009693] Sources: GOC:tair_curators Definition: Any process that activates or increases the frequency, rate or extent of an ethylene biosynthetic process.